{
  "term_label": "DNA binding",
  "gene": "UniProtKB:Q9H211",
  "gene_name": "DNA replication factor Cdt1",
  "gene_symbol": "CDT1",
  "term_id": "GO:0003677"
}